{
  "gene_symbol": "A0A0G2JN53",
  "term_id": "UNKNOWN:0002",
  "gene_name": "IQ motif and SEC7 domain-containing protein 3",
  "term_label": "Unknown biological process",
  "gene": "UniProtKB:A0A0G2JN53"
}